{
  "gene_symbol": "NCF1",
  "term_label": "respiratory burst",
  "term_id": "GO:0045730",
  "gene": "UniProtKB:P14598",
  "gene_name": "Neutrophil cytosol factor 1"
}